{
  "gene_symbol": "WLS",
  "term_id": "GO:0006886",
  "gene": "UniProtKB:Q5T9L3",
  "gene_name": "Protein wntless homolog",
  "term_label": "intracellular protein transport"
}